{
  "term_id": "GO:0005125",
  "gene_name": "Protein Wnt-16",
  "gene_symbol": "WNT16",
  "gene": "UniProtKB:Q9UBV4",
  "term_label": "cytokine activity"
}